{
  "gene_name": "Homeobox protein Hox-B9",
  "gene_symbol": "HOXB9",
  "gene": "UniProtKB:P17482",
  "term_id": "GO:0005634",
  "term_label": "nucleus"
}